negative regulation of synergid differentiation [GO:0045698] (biological process) Definition: Any process that stops, prevents, or reduces the frequency, rate or extent of synergid cell differentiation. Sources: GOC:go_curators Also known as: down regulation of synergid differentiation, down-regulation of synergid differentiation, downregulation of synergid differentiation, negative regulation of synergid cell differentiation, inhibition of synergid differentiation Relationships: is a type of negative regulation of cell differentiation [GO:0045596]; is_a regulation of synergid differentiation [GO:0045697]; is a type of negative regulation of multicellular organismal process [GO:0051241]; negatively regulates GO:0009563